{
  "gene_symbol": "RASGRP1",
  "term_label": "plasma membrane",
  "gene": "UniProtKB:O95267",
  "gene_name": "RAS guanyl-releasing protein 1",
  "term_id": "GO:0005886"
}